{
  "term_label": "glutamate receptor signaling pathway",
  "gene_name": "Guanine nucleotide-binding protein G(q) subunit alpha",
  "gene": "UniProtKB:P50148",
  "term_id": "GO:0007215",
  "gene_symbol": "GNAQ"
}